{
  "term_label": "protein processing",
  "gene": "UniProtKB:Q9Y6L7",
  "gene_symbol": "TLL2",
  "term_id": "GO:0016485",
  "gene_name": "Tolloid-like protein 2"
}